{
  "term_label": "cytosol",
  "gene_name": "Peroxiredoxin-6",
  "gene_symbol": "PRDX6",
  "gene": "UniProtKB:P30041",
  "term_id": "GO:0005829"
}